{
  "gene_symbol": "BIRC7",
  "gene": "UniProtKB:Q96CA5",
  "term_label": "cytoplasm",
  "term_id": "GO:0005737",
  "gene_name": "Baculoviral IAP repeat-containing protein 7"
}